bud dormancy process [GO:0097207] (biological process) Note: Bud dormancy may precede dormancy of the whole plant. Relationships: is a type of dormancy process [GO:0022611]; is a type of multicellular organismal process [GO:0032501] Definition: A dormancy process in which dormancy (sometimes called a dormant state) is induced, maintained or broken in a bud. Bud dormancy is a suspension of most physiological activity and growth that can be reactivated. It may be a response to environmental conditions such as seasonality or extreme heat, drought, or cold. The exit from bud dormancy is marked by the resumed growth of the bud. Sources: GOC:PO_curators, PO_REF:00009 Also known as: bud dormancy